{
  "gene_symbol": "ZBTB12",
  "term_id": "GO:0005654",
  "term_label": "nucleoplasm",
  "gene_name": "Zinc finger and BTB domain-containing protein 12",
  "gene": "UniProtKB:Q9Y330"
}